manganese ion transmembrane transporter activity [GO:0005384] (molecular function) Definition: Enables the transfer of manganese (Mn) ions from one side of a membrane to the other. Subtypes: manganese:proton antiporter activity [GO:0010486], ABC-type manganese transporter activity [GO:0015410], P-type manganese transporter activity [GO:0140613], calcium:manganese antiporter activity [GO:0140983] Sources: GOC:dgf Relationships: is a type of transition metal ion transmembrane transporter activity [GO:0046915]; is part of GO:0071421